{
  "term_label": "Unknown biological process",
  "gene_name": "Delta and Notch-like epidermal growth factor-related receptor",
  "gene": "UniProtKB:Q8NFT8",
  "gene_symbol": "DNER",
  "term_id": "UNKNOWN:0002"
}